{
  "term_label": "Unknown molecular function",
  "gene_symbol": "TRAV25",
  "term_id": "UNKNOWN:0001",
  "gene_name": "T cell receptor alpha variable 25",
  "gene": "UniProtKB:A0A0B4J276"
}